{
  "gene": "UniProtKB:O60565",
  "term_label": "BMP binding",
  "gene_symbol": "GREM1",
  "gene_name": "Gremlin-1",
  "term_id": "GO:0036122"
}